{
  "term_id": "GO:0055085",
  "gene_symbol": "SLC35E2B",
  "gene_name": "Solute carrier family 35 member E2B",
  "term_label": "transmembrane transport",
  "gene": "UniProtKB:P0CK96"
}